glycosphingolipid catabolic process [GO:0046479] (biological process) Sources: ISBN:0198506732 Definition: The chemical reactions and pathways resulting in the breakdown of glycosphingolipid, a compound with residues of sphingoid and at least one monosaccharide. Relationships: is a type of GO:0006687; is a type of glycolipid catabolic process [GO:0019377]; is a type of sphingolipid catabolic process [GO:0030149] Subtypes: ganglioside catabolic process [GO:0006689], glycosylceramide catabolic process [GO:0046477] Also known as: glycosphingolipid breakdown, glycosphingolipid catabolism, glycosphingolipid degradation